kinocilium [GO:0060091] (cellular component) References: PMID:15882574 Sources: GOC:cilia, GOC:dph Relationships: is a type of neuron projection [GO:0043005]; is a type of 9+2 non-motile cilium [GO:0097732]; is part of stereocilium bundle [GO:0032421]; is part of organelle [GO:0043226]; has part radial spoke [GO:0001534] Definition: A nonmotile primary cilium that is found at the apical surface of auditory receptor cells. The kinocilium is surrounded by actin-based stereocilia.